regulation of modification of synapse structure, modulating synaptic transmission [GO:0098987] (biological process) Definition: Any process that regulates the modification of synaptic structure and as a result regulates synaptic transmission. Relationships: is a type of modulation of chemical synaptic transmission [GO:0050804]; is a type of regulation of modification of synaptic structure [GO:1905244] Note: Note that this term was created for the SynGO project, and will be obsoleted when the SynGO annotations are made in Noctua. Sources: GOC:dos